{
  "term_id": "GO:0045454",
  "gene": "UniProtKB:Q16881",
  "gene_symbol": "TXNRD1",
  "term_label": "cell redox homeostasis",
  "gene_name": "Thioredoxin reductase 1, cytoplasmic"
}